positive regulation of syncytium formation by plasma membrane fusion [GO:0060143] (biological process) Subtypes: positive regulation of macrophage fusion [GO:0034241], positive regulation of myoblast fusion [GO:1901741] Definition: Any process that increases the frequency, rate or extent of the formation of a syncytium, a mass of cytoplasm containing several nuclei enclosed within a single plasma membrane, by the fusion of the plasma membranes of two or more individual cells. Relationships: is a type of positive regulation of developmental process [GO:0051094]; is a type of positive regulation of cellular component organization [GO:0051130]; is a type of regulation of syncytium formation by plasma membrane fusion [GO:0060142]; RO_0002213 syncytium formation by plasma membrane fusion [GO:0000768] Sources: GOC:dph